{
  "gene_name": "ATPase family AAA domain-containing protein 3A",
  "gene_symbol": "ATAD3A",
  "gene": "UniProtKB:Q9NVI7",
  "term_label": "mitochondrion",
  "term_id": "GO:0005739"
}